R7 cell differentiation [GO:0045466] (biological process) Definition: The process in which a relatively unspecialized cell acquires the specialized features of the R7 photoreceptor. References: PMID:11880339 Relationships: is_a compound eye photoreceptor cell differentiation [GO:0001751] Regulation: regulated by regulation of R7 cell differentiation [GO:0045676]; RO_0002212 by GO:0045677; positively regulated by positive regulation of R7 cell differentiation [GO:0045678]